{
  "term_label": "plasma membrane",
  "gene_name": "Potassium voltage-gated channel subfamily H member 3",
  "term_id": "GO:0005886",
  "gene": "UniProtKB:Q9ULD8",
  "gene_symbol": "KCNH3"
}